{
  "gene_name": "Alpha-2-macroglobulin receptor-associated protein",
  "term_id": "GO:0012505",
  "gene": "UniProtKB:P30533",
  "gene_symbol": "LRPAP1",
  "term_label": "endomembrane system"
}